{
  "term_id": "GO:0004674",
  "term_label": "protein serine/threonine kinase activity",
  "gene_symbol": "NIM1K",
  "gene_name": "Serine_threonine-protein kinase NIM1",
  "gene": "UniProtKB:Q8IY84"
}